{
  "gene_symbol": "UBE4A",
  "term_id": "GO:0005634",
  "gene": "UniProtKB:Q14139",
  "term_label": "nucleus",
  "gene_name": "Ubiquitin conjugation factor E4 A"
}